MdtBC Complex [GO:1990203] (cellular component) Relationships: is a type of GO:0098797; is_a transmembrane transporter complex [GO:1902495] Also known as: multidrug efflux pump MdtBC Definition: A protein complex containing two transmembrane subunits; a MdtB dimer and one unit of MdtC. Capable of exporting substrates across the cell membrane. Involved in conferring antibiotic resistance of Gram-negative bacteria by transporting drugs across the membrane. References: PMID:20038594 Sources: GOC:bhm